{
  "gene_symbol": "HERC5",
  "term_label": "ubiquitin-dependent protein catabolic process",
  "gene": "UniProtKB:Q9UII4",
  "term_id": "GO:0006511",
  "gene_name": "E3 ISG15--protein ligase HERC5"
}